{
  "gene_symbol": "MZT1",
  "term_id": "GO:0005813",
  "gene_name": "Mitotic-spindle organizing protein 1",
  "term_label": "centrosome",
  "gene": "UniProtKB:Q08AG7"
}